mitochondrion-associated adherens complex [GO:0097423] (cellular component) Also known as: mitochondrial adhaerens complex, MAC References: PMID:20089910 Sources: NIF_Subcellular:sao1933817066 Definition: An organelle arrangement comprised of the following elements: a mitochondrion positioned near the presynaptic membrane; an electron-dense mitochondrial plaque adjacent to the outer mitochondrial membrane that faces the presynaptic membrane; filament-like elements appearing to link the mitochondrial plaque to a cell-cell junction region (sometimes termed punctum adherens); tubular or vesicular-appearing membrane (also called vesicular chain) interposed among the filaments. Mitochondrion-associated adherens complexes were initially described in the dorsal horn of the spinal cord. They are found in calyces and other large terminals of the auditory brainstem, and in a variety of mammalian species including humans. Relationships: is a type of cellular anatomical structure [GO:0110165]; BFO_0000051 GO:0005739; has part cell-cell junction [GO:0005911]